{
  "term_label": "GTPase activator activity",
  "gene_symbol": "ARHGAP12",
  "term_id": "GO:0005096",
  "gene_name": "Rho GTPase-activating protein 12",
  "gene": "UniProtKB:Q8IWW6"
}